negative regulation of flavonol biosynthetic process [GO:1900385] (biological process) Also known as: down regulation of flavonol biosynthetic process, down-regulation of flavonol biosynthetic process, downregulation of flavonol biosynthetic process, inhibition of flavonol biosynthetic process Sources: GOC:TermGenie Definition: Any process that stops, prevents or reduces the frequency, rate or extent of flavonol biosynthetic process. Relationships: is a type of negative regulation of flavonoid biosynthetic process [GO:0009964]; is a type of regulation of flavonol biosynthetic process [GO:1900384]; negatively regulates GO:0051555